{
  "gene": "UniProtKB:Q9NSY2",
  "gene_symbol": "STARD5",
  "term_id": "GO:0070508",
  "term_label": "cholesterol import",
  "gene_name": "StAR-related lipid transfer protein 5"
}